{
  "gene_name": "T cell receptor alpha variable 8-3",
  "gene_symbol": "TRAV8-3",
  "gene": "UniProtKB:A0A0A6YYJ7",
  "term_label": "adaptive immune response",
  "term_id": "GO:0002250"
}